positive regulation of hepatic stellate cell migration [GO:0061870] (biological process) References: PMID:24204762 Definition: Any process that increases the frequency, rate or extent of hepatic stellate cell migration. Relationships: is a type of positive regulation of fibroblast migration [GO:0010763]; is a type of regulation of hepatic stellate cell migration [GO:0061869]; positively regulates GO:0061868